{
  "term_label": "ubiquitin protein ligase activity",
  "gene": "UniProtKB:Q495X7",
  "gene_name": "Tripartite motif-containing protein 60",
  "gene_symbol": "TRIM60",
  "term_id": "GO:0061630"
}